{
  "term_id": "GO:0030527",
  "gene_name": "Histone H2B type 1-A",
  "gene": "UniProtKB:Q96A08",
  "term_label": "structural constituent of chromatin",
  "gene_symbol": "H2BC1"
}